{
  "gene_name": "Microtubule-associated protein RP_EB family member 3",
  "gene": "UniProtKB:Q9UPY8",
  "gene_symbol": "MAPRE3",
  "term_label": "spindle midzone",
  "term_id": "GO:0051233"
}